GINS complex [GO:0000811] (cellular component) Definition: A heterotetrameric protein complex that associates with replication origins, where it is required for the initiation of DNA replication, and with replication forks. References: PMID:12730134, PMID:16990792, PMID:17467990 Sources: GOC:rb, GOC:rn Also known as: Go, Ichi, Ni and San complex Relationships: is a type of GO:0031261; BFO_0000050 nuclear chromosome [GO:0000228]